epithelial cell differentiation involved in prostate gland development [GO:0060742] (biological process) Definition: The process in which a relatively unspecialized cell acquires specialized features of an epithelial cell of the prostate gland. Sources: GOC:dph Relationships: is a type of developmental process involved in reproduction [GO:0003006]; is a type of epithelial cell differentiation [GO:0030855]; is part of prostate gland development [GO:0030850] Subtypes: secretory columnal luminar epithelial cell differentiation involved in prostate glandular acinus development [GO:0060528], squamous basal epithelial stem cell differentiation involved in prostate gland acinus development [GO:0060529], neuroendocrine cell differentiation involved in prostate gland acinus development [GO:0060531]